neural crest cell migration [GO:0001755] (biological process) Relationships: is a type of mesenchymal cell migration [GO:0090497]; BFO_0000050 GO:0014032 Sources: GOC:ascb_2009, GOC:dph, GOC:tb, ISBN:0878932437 Definition: The characteristic movement of cells from the dorsal ridge of the neural tube to a variety of locations in a vertebrate embryo. Subtypes: neural crest cell migration involved in heart formation [GO:0003147], cardiac neural crest cell migration involved in outflow tract morphogenesis [GO:0003253], GO:0036484, GO:1901166